{
  "gene": "UniProtKB:Q15014",
  "term_id": "UNKNOWN:0001",
  "term_label": "Unknown molecular function",
  "gene_symbol": "MORF4L2",
  "gene_name": "Mortality factor 4-like protein 2"
}